{
  "gene": "UniProtKB:P12830",
  "term_label": "flotillin complex",
  "gene_symbol": "CDH1",
  "term_id": "GO:0016600",
  "gene_name": "Cadherin-1"
}